mitochondrial outer membrane translocase complex [GO:0005742] (cellular component) Definition: A large complex of the mitochondrial outer membrane that mediates transport of proteins into all mitochondrial compartments. References: PMID:12581629 Relationships: is a type of GO:0098799 Subtypes: SAM complex [GO:0001401], GO:0140596 Also known as: mitochondrion outer membrane translocase complex, GIP complex